{
  "term_label": "Unknown biological process",
  "gene_name": "Trafficking protein particle complex subunit 13",
  "gene_symbol": "TRAPPC13",
  "term_id": "UNKNOWN:0002",
  "gene": "UniProtKB:A5PLN9"
}